{
  "term_label": "keratin filament",
  "term_id": "GO:0045095",
  "gene": "UniProtKB:Q5XKE5",
  "gene_name": "Keratin, type II cytoskeletal 79",
  "gene_symbol": "KRT79"
}